{
  "gene_name": "Cytosolic carboxypeptidase 6",
  "term_id": "GO:0015630",
  "gene": "UniProtKB:Q5VU57",
  "term_label": "microtubule cytoskeleton",
  "gene_symbol": "AGBL4"
}